{
  "gene_symbol": "MSANTD3",
  "term_id": "UNKNOWN:0002",
  "term_label": "Unknown biological process",
  "gene_name": "Myb_SANT-like DNA-binding domain-containing protein 3",
  "gene": "UniProtKB:Q96H12"
}